{
  "gene_name": "Interferon-induced, double-stranded RNA-activated protein kinase",
  "term_id": "GO:0004694",
  "gene_symbol": "EIF2AK2",
  "gene": "UniProtKB:P19525",
  "term_label": "eukaryotic translation initiation factor 2alpha kinase activity"
}